histone H4K16 deacetylase activity, hydrolytic mechanism [GO:0034739] (molecular function) Also known as: histone H4K12 deacetylase activity, histone H4-K16 deacetylase activity, histone deacetylase activity (H4-K16 specific) Relationships: is a type of histone H4K deacetylase activity [GO:0141051]; is a type of GO:0141221 Definition: Catalysis of the reaction: histone H4 N6-acetyl-L-lysine (position 16) + H2O = histone H4 L-lysine (position 16) + acetate. This reaction represents the removal of an acetyl group from lysine at position 16 of the histone H4 protein. References: PMID:28450737 Sources: GOC:vw Note: Note that the residue position corresponds to the canonical human H4 histone (UniProtKB:P02309); this residue is conserved across all eukaryotes. Note that the initiation methionine is cleaved, so the first residue is S1.